positive regulation of bile acid biosynthetic process [GO:0070859] (biological process) Also known as: positive regulation of bile acid anabolism, positive regulation of bile acid biosynthesis, positive regulation of bile acid formation, positive regulation of bile acid synthesis, up regulation of bile acid biosynthetic process, up-regulation of bile acid biosynthetic process, upregulation of bile acid biosynthetic process, activation of bile acid biosynthetic process, stimulation of bile acid biosynthetic process Definition: Any process that activates or increases the frequency, rate or extent of the chemical reactions and pathways resulting in the formation of bile acids. Relationships: is a type of positive regulation of steroid biosynthetic process [GO:0010893]; is a type of positive regulation of small molecule metabolic process [GO:0062013]; is_a regulation of bile acid biosynthetic process [GO:0070857]; positively regulates bile acid biosynthetic process [GO:0006699] Sources: GOC:BHF, GOC:mah